{
  "gene_symbol": "FOXI3",
  "term_id": "GO:0000981",
  "term_label": "DNA-binding transcription factor activity, RNA polymerase II-specific",
  "gene_name": "Forkhead box protein I3",
  "gene": "UniProtKB:A8MTJ6"
}